cell proliferation involved in outflow tract morphogenesis [GO:0061325] (BP) Definition: The multiplication or reproduction of cells, resulting in the expansion of a cell population that contributes to the shaping of the outflow tract. Sources: GOC:dph, GOC:mtg_heart Relationships: is a type of cell proliferation involved in heart morphogenesis [GO:0061323]; BFO_0000050 outflow tract morphogenesis [GO:0003151] Regulation: regulated by regulation of cell proliferation involved in outflow tract morphogenesis [GO:1901963]; positively regulated by positive regulation of cell proliferation involved in outflow tract morphogenesis [GO:1901964]